{
  "gene_symbol": "PARP10",
  "term_id": "GO:0005737",
  "gene": "UniProtKB:Q53GL7",
  "term_label": "cytoplasm",
  "gene_name": "Protein mono-ADP-ribosyltransferase PARP10"
}